{
  "gene": "UniProtKB:Q9NXE4",
  "gene_symbol": "SMPD4",
  "term_id": "GO:0006685",
  "term_label": "sphingomyelin catabolic process",
  "gene_name": "Sphingomyelin phosphodiesterase 4"
}